{
  "gene_symbol": "MGST3",
  "term_id": "GO:0004364",
  "gene_name": "Glutathione S-transferase 3, mitochondrial",
  "term_label": "glutathione transferase activity",
  "gene": "UniProtKB:O14880"
}